{
  "term_label": "glucuronosyl-N-acetylgalactosaminyl-proteoglycan 4-beta-N-acetylgalactosaminyltransferase activity",
  "gene_symbol": "CHPF",
  "term_id": "GO:0047238",
  "gene": "UniProtKB:Q8IZ52",
  "gene_name": "Chondroitin sulfate synthase 2"
}